transcription factor TFIIE complex [GO:0005673] (CC) References: PMID:16547462 Sources: GOC:jl Relationships: is_a GO:0090575; is part of RNA polymerase II, holoenzyme [GO:0016591] Definition: A transcription factor which in humans consists of a complex of two alpha and two beta chains. Recruits TFIIH to the initiation complex and helps activate both RNA polymerase II and TFIIH.